{
  "term_id": "GO:0005744",
  "gene": "UniProtKB:Q3ZCQ8",
  "gene_symbol": "TIMM50",
  "term_label": "TIM23 mitochondrial import inner membrane translocase complex",
  "gene_name": "Mitochondrial import inner membrane translocase subunit TIM50"
}